regulation of defecation [GO:2000292] (biological process) Relationships: is a type of regulation of digestive system process [GO:0044058]; is a type of regulation of excretion [GO:0044062]; regulates defecation [GO:0030421] Subtypes: negative regulation of defecation [GO:2000293], positive regulation of defecation [GO:2000294], GO:2000746 Sources: GOC:obol Definition: Any process that modulates the frequency, rate or extent of defecation.